{
  "gene_symbol": "BLVRB",
  "gene_name": "Flavin reductase (NADPH)",
  "gene": "UniProtKB:P30043",
  "term_id": "UNKNOWN:0002",
  "term_label": "Unknown biological process"
}